{
  "term_id": "GO:0006354",
  "gene": "UniProtKB:Q9NW08",
  "gene_name": "DNA-directed RNA polymerase III subunit RPC2",
  "term_label": "DNA-templated transcription elongation",
  "gene_symbol": "POLR3B"
}